{
  "gene_name": "Galectin-3-binding protein",
  "term_id": "UNKNOWN:0001",
  "gene": "UniProtKB:Q08380",
  "gene_symbol": "LGALS3BP",
  "term_label": "Unknown molecular function"
}